{
  "gene_symbol": "SLC16A1",
  "gene_name": "Monocarboxylate transporter 1",
  "term_id": "GO:0016323",
  "gene": "UniProtKB:P53985",
  "term_label": "basolateral plasma membrane"
}